{
  "gene_name": "Peptidyl-tRNA hydrolase 2, mitochondrial",
  "gene_symbol": "PTRH2",
  "term_id": "GO:2000210",
  "gene": "UniProtKB:Q9Y3E5",
  "term_label": "positive regulation of anoikis"
}